{
  "gene_symbol": "LEO1",
  "term_id": "GO:1990269",
  "gene": "UniProtKB:Q8WVC0",
  "term_label": "RNA polymerase II C-terminal domain phosphoserine binding",
  "gene_name": "RNA polymerase-associated protein LEO1"
}